{
  "gene_symbol": "PUS1",
  "term_label": "mRNA pseudouridine synthesis",
  "gene": "UniProtKB:Q9Y606",
  "term_id": "GO:1990481",
  "gene_name": "Pseudouridylate synthase 1 homolog"
}